{
  "term_id": "UNKNOWN:0002",
  "gene_name": "Proline-rich protein 12",
  "term_label": "Unknown biological process",
  "gene_symbol": "PRR12",
  "gene": "UniProtKB:Q9ULL5"
}